{
  "gene_name": "BEN domain-containing protein 7",
  "term_id": "UNKNOWN:0001",
  "gene": "UniProtKB:Q8N7W2",
  "gene_symbol": "BEND7",
  "term_label": "Unknown molecular function"
}